{
  "gene_symbol": "BRWD3",
  "gene": "UniProtKB:Q6RI45",
  "term_id": "GO:0008360",
  "gene_name": "Bromodomain and WD repeat-containing protein 3",
  "term_label": "regulation of cell shape"
}